{
  "gene_name": "Selenide, water dikinase 1",
  "term_label": "selenocysteine biosynthetic process",
  "gene": "UniProtKB:P49903",
  "gene_symbol": "SEPHS1",
  "term_id": "GO:0016260"
}